{
  "gene_symbol": "TMEM108",
  "term_id": "GO:0097106",
  "gene_name": "Transmembrane protein 108",
  "gene": "UniProtKB:Q6UXF1",
  "term_label": "postsynaptic density organization"
}